{
  "term_id": "GO:0019722",
  "gene_name": "Atypical chemokine receptor 3",
  "gene_symbol": "ACKR3",
  "term_label": "calcium-mediated signaling",
  "gene": "UniProtKB:P25106"
}